{
  "gene": "UniProtKB:O43852",
  "term_id": "UNKNOWN:0002",
  "term_label": "Unknown biological process",
  "gene_name": "Calumenin",
  "gene_symbol": "CALU"
}